{
  "term_id": "UNKNOWN:0002",
  "gene": "UniProtKB:Q8N1A0",
  "gene_name": "Keratin-like protein KRT222",
  "term_label": "Unknown biological process",
  "gene_symbol": "KRT222"
}